{
  "gene_name": "Ribosome biogenesis protein BOP1",
  "term_label": "ribonucleoprotein complex binding",
  "gene": "UniProtKB:Q14137",
  "term_id": "GO:0043021",
  "gene_symbol": "BOP1"
}